{
  "term_id": "GO:0002244",
  "gene_name": "Tumor necrosis factor receptor superfamily member 13B",
  "gene": "UniProtKB:O14836",
  "term_label": "hematopoietic progenitor cell differentiation",
  "gene_symbol": "TNFRSF13B"
}